positive regulation of septation initiation signaling [GO:0031031] (biological process) Sources: GOC:mah Definition: Any process that activates or increases the frequency, rate or extent of septation initiation signaling. Also known as: positive regulation of septation initiation network, positive regulation of septation initiation signalling, up regulation of septation initiation signaling, up-regulation of septation initiation signaling, upregulation of septation initiation signaling, activation of septation initiation signaling, stimulation of septation initiation signaling, positive regulation of septation initiation signaling cascade Relationships: is a type of GO:0010973; is_a regulation of septation initiation signaling [GO:0031029]; is a type of positive regulation of small GTPase mediated signal transduction [GO:0051057]; positively regulates GO:0031028